{
  "term_id": "GO:0000974",
  "gene_name": "Pre-mRNA-splicing factor ISY1 homolog",
  "term_label": "Prp19 complex",
  "gene_symbol": "ISY1",
  "gene": "UniProtKB:Q9ULR0"
}